{
  "term_label": "Unknown biological process",
  "gene_symbol": "DCAF12L2",
  "gene_name": "DDB1- and CUL4-associated factor 12-like protein 2",
  "term_id": "UNKNOWN:0002",
  "gene": "UniProtKB:Q5VW00"
}